{
  "term_label": "negative regulation of inflammatory response",
  "gene_name": "C-X-C motif chemokine 17",
  "gene": "UniProtKB:Q6UXB2",
  "term_id": "GO:0050728",
  "gene_symbol": "CXCL17"
}